dATP catabolic process [GO:0046061] (biological process) Definition: The chemical reactions and pathways resulting in the breakdown of dATP, deoxyadenosine triphosphate (2'-deoxyadenosine 5'-triphosphate). Sources: GOC:go_curators Also known as: dATP breakdown, dATP catabolism, dATP degradation Relationships: is a type of purine deoxyribonucleotide catabolic process [GO:0009155]; is a type of purine deoxyribonucleoside triphosphate catabolic process [GO:0009217]; is a type of dATP metabolic process [GO:0046060]